regulation of border follicle cell delamination [GO:0030710] (biological process) Definition: Any process that regulates the frequency, rate or extent of border cell delamination. Relationships: is a type of GO:0022407; regulates border follicle cell delamination [GO:0030709] Subtypes: positive regulation of border follicle cell delamination [GO:0030711], negative regulation of border follicle cell delamination [GO:0030712] Also known as: regulation of border cell delamination References: PMID:10822261